{
  "term_label": "maturation of LSU-rRNA from tricistronic rRNA transcript (SSU-rRNA, 5.8S rRNA, LSU-rRNA)",
  "term_id": "GO:0000463",
  "gene_symbol": "DDX18",
  "gene": "UniProtKB:Q9NVP1",
  "gene_name": "ATP-dependent RNA helicase DDX18"
}